{
  "gene_name": "Testis-expressed protein 26",
  "term_label": "Unknown molecular function",
  "term_id": "UNKNOWN:0001",
  "gene": "UniProtKB:Q8N6G2",
  "gene_symbol": "TEX26"
}